poly(G) binding [GO:0034046] (molecular function) Also known as: poly(G) binding, within an RNA molecule, poly(rG) binding Definition: Binding to a sequence of guanine residues in an RNA molecule. Relationships: is a type of poly-purine tract binding [GO:0070717] Sources: GOC:mah